{
  "term_id": "GO:0019221",
  "gene_symbol": "STAT6",
  "gene": "UniProtKB:P42226",
  "gene_name": "Signal transducer and activator of transcription 6",
  "term_label": "cytokine-mediated signaling pathway"
}